{
  "term_label": "phosphatidylinositol-4-phosphate binding",
  "gene_name": "Golgi phosphoprotein 3",
  "gene": "UniProtKB:Q9H4A6",
  "gene_symbol": "GOLPH3",
  "term_id": "GO:0070273"
}